{
  "term_label": "spermatogenesis",
  "gene": "UniProtKB:Q96EP5",
  "gene_symbol": "DAZAP1",
  "term_id": "GO:0007283",
  "gene_name": "DAZ-associated protein 1"
}